regulation of antigen processing and presentation of peptide antigen [GO:0002583] (biological process) Definition: Any process that modulates the frequency, rate, or extent of antigen processing and presentation of peptide antigen. Also known as: regulation of peptide antigen processing and presentation Subtypes: negative regulation of antigen processing and presentation of peptide antigen [GO:0002584], positive regulation of antigen processing and presentation of peptide antigen [GO:0002585], regulation of antigen processing and presentation of peptide antigen via MHC class II [GO:0002586], regulation of antigen processing and presentation of peptide antigen via MHC class I [GO:0002589], regulation of antigen processing and presentation of peptide antigen via MHC class Ib [GO:0002595], regulation of peptide antigen transport [GO:1901039] Relationships: is a type of regulation of antigen processing and presentation [GO:0002577]; regulates antigen processing and presentation of peptide antigen [GO:0048002] Sources: GOC:add